{
  "gene": "UniProtKB:Q92608",
  "term_label": "small GTPase binding",
  "term_id": "GO:0031267",
  "gene_symbol": "DOCK2",
  "gene_name": "Dedicator of cytokinesis protein 2"
}